{
  "term_id": "GO:0003735",
  "term_label": "structural constituent of ribosome",
  "gene_symbol": "RPL31",
  "gene_name": "Large ribosomal subunit protein eL31",
  "gene": "UniProtKB:P62899"
}